{
  "gene": "UniProtKB:Q3MIV0",
  "gene_symbol": "KRTAP22-1",
  "term_label": "Unknown biological process",
  "gene_name": "Keratin-associated protein 22-1",
  "term_id": "UNKNOWN:0002"
}